{
  "gene_symbol": "EFCAB11",
  "gene": "UniProtKB:Q9BUY7",
  "term_id": "GO:0030234",
  "gene_name": "EF-hand calcium-binding domain-containing protein 11",
  "term_label": "enzyme regulator activity"
}